{
  "gene_name": "Cartilage intermediate layer protein 1",
  "gene_symbol": "CILP",
  "term_label": "Unknown biological process",
  "term_id": "UNKNOWN:0002",
  "gene": "UniProtKB:O75339"
}